{
  "term_id": "UNKNOWN:0001",
  "gene": "UniProtKB:Q9BRP9",
  "gene_name": "Putative uncharacterized protein MGC13053",
  "gene_symbol": "Q9BRP9",
  "term_label": "Unknown molecular function"
}